{
  "term_id": "GO:0005886",
  "gene_name": "Carcinoembryonic antigen-related cell adhesion molecule 20",
  "gene_symbol": "CEACAM20",
  "term_label": "plasma membrane",
  "gene": "UniProtKB:Q6UY09"
}